{
  "gene_name": "Sperm-associated antigen 7",
  "gene": "UniProtKB:O75391",
  "term_label": "Unknown cellular component",
  "term_id": "UNKNOWN:0003",
  "gene_symbol": "SPAG7"
}